midbrain-hindbrain boundary maturation during neural plate development [GO:0022005] (biological process) Definition: A developmental process occurring before the brain has been specified along the neural axis that is required for the midbrain-hindbrain boundary to attain its fully functional state. The midbrain-hindbrain domain of the embryonic brain is comprised of the mesencephalic vesicle and the first rhombencephalic vesicle at early somitogenesis stages. An organizing center at the boundary patterns the midbrain and hindbrain primordia of the neural plate. References: PMID:15541513 Sources: GOC:cls, GOC:dgh, GOC:dph, GOC:jid, GO_REF:0000021 Also known as: midbrain-hindbrain boundary maturation involved in neural plate development Relationships: is a type of multicellular organismal process [GO:0032501]; is part of GO:0021732